telomere maintenance via telomere trimming [GO:0090737] (biological process) Relationships: is a type of telomere maintenance [GO:0000723] References: PMID:27918544 Sources: GOC:BHF, GOC:BHF_telomere, GOC:nc Definition: A process that contributes to the maintenance of proper telomeric length and structure via the activation of telomere shortening pathways that compensate telomerase-dependent excessive telomere elongation. Telomere attrition is mediated by a mechanism which involves the generation of single-stranded C-rich telomeric DNA, and the formation and removal of double-stranded telomeric circular DNA (T-circles). Telomere trimming is an independent pathway to recombination-mediated telomere elongation and the well-documented gradual telomere attrition that accompanies cellular replication.